{
  "gene": "UniProtKB:Q96CP7",
  "gene_symbol": "TLCD1",
  "term_label": "Unknown molecular function",
  "gene_name": "TLC domain-containing protein 1",
  "term_id": "UNKNOWN:0001"
}